{
  "term_label": "Unknown cellular component",
  "gene_symbol": "GFY",
  "gene_name": "Golgi-associated olfactory signaling regulator",
  "term_id": "UNKNOWN:0003",
  "gene": "UniProtKB:I3L273"
}